{
  "gene_symbol": "RBMXL2",
  "gene": "UniProtKB:O75526",
  "term_id": "UNKNOWN:0003",
  "gene_name": "RNA-binding motif protein, X-linked-like-2",
  "term_label": "Unknown cellular component"
}